{
  "gene": "UniProtKB:Q99946",
  "term_label": "synapse organization",
  "gene_name": "Proline-rich transmembrane protein 1",
  "term_id": "GO:0050808",
  "gene_symbol": "PRRT1"
}